{
  "gene": "UniProtKB:Q8WW34",
  "gene_name": "Transmembrane protein 239",
  "gene_symbol": "TMEM239",
  "term_label": "Unknown cellular component",
  "term_id": "UNKNOWN:0003"
}